{
  "gene_symbol": "NEMP1",
  "gene_name": "Nuclear envelope integral membrane protein 1",
  "term_id": "GO:0005635",
  "term_label": "nuclear envelope",
  "gene": "UniProtKB:O14524"
}